{
  "gene_name": "Tumor necrosis factor-inducible gene 6 protein",
  "term_id": "GO:0050728",
  "gene": "UniProtKB:P98066",
  "gene_symbol": "TNFAIP6",
  "term_label": "negative regulation of inflammatory response"
}